negative regulation of cordyol C biosynthetic process [GO:1900862] (biological process) Sources: GOC:TermGenie, GOC:di Also known as: down regulation of cordyol C biosynthetic process, down-regulation of cordyol C biosynthetic process, downregulation of cordyol C biosynthetic process Definition: Any process that stops, prevents or reduces the frequency, rate or extent of cordyol C biosynthetic process. Relationships: is a type of negative regulation of secondary metabolite biosynthetic process [GO:1900377]; is_a GO:1900861; negatively regulates GO:1900799